{
  "gene_symbol": "BNIP2",
  "gene": "UniProtKB:Q12982",
  "term_label": "cytoplasm",
  "gene_name": "BCL2_adenovirus E1B 19 kDa protein-interacting protein 2",
  "term_id": "GO:0005737"
}